{
  "term_id": "GO:0016567",
  "gene_name": "E3 ubiquitin-protein ligase MARCHF3",
  "gene": "UniProtKB:Q86UD3",
  "term_label": "protein ubiquitination",
  "gene_symbol": "MARCHF3"
}